{
  "term_id": "GO:0046033",
  "term_label": "AMP metabolic process",
  "gene_name": "AMP deaminase 1",
  "gene_symbol": "AMPD1",
  "gene": "UniProtKB:P23109"
}